{
  "term_id": "UNKNOWN:0002",
  "gene_symbol": "SPDYE10",
  "gene_name": "Speedy protein E10",
  "gene": "UniProtKB:P0DUX0",
  "term_label": "Unknown biological process"
}